{
  "gene_symbol": "KBTBD2",
  "term_label": "proteasome-mediated ubiquitin-dependent protein catabolic process",
  "term_id": "GO:0043161",
  "gene_name": "Kelch repeat and BTB domain-containing protein 2",
  "gene": "UniProtKB:Q8IY47"
}